{
  "term_label": "cyclosporin A binding",
  "gene_name": "Peptidyl-prolyl cis-trans isomerase G",
  "gene_symbol": "PPIG",
  "gene": "UniProtKB:Q13427",
  "term_id": "GO:0016018"
}